{
  "term_id": "GO:0006887",
  "gene": "UniProtKB:O15127",
  "gene_name": "Secretory carrier-associated membrane protein 2",
  "gene_symbol": "SCAMP2",
  "term_label": "exocytosis"
}